{
  "gene": "UniProtKB:Q9NZD1",
  "gene_symbol": "GPRC5D",
  "gene_name": "G-protein coupled receptor family C group 5 member D",
  "term_label": "extracellular exosome",
  "term_id": "GO:0070062"
}